{
  "gene_symbol": "CPLX3",
  "gene_name": "Complexin-3",
  "gene": "UniProtKB:Q8WVH0",
  "term_label": "SNARE complex",
  "term_id": "GO:0031201"
}